{
  "gene_name": "Cyclin-dependent kinase 9",
  "term_label": "nucleus",
  "gene_symbol": "CDK9",
  "gene": "UniProtKB:P50750",
  "term_id": "GO:0005634"
}